sensory organ precursor cell division [GO:0045035] (biological process) References: PMID:11171389, PMID:18295597 Sources: GOC:mah Also known as: sense organ precursor cell division Definition: The series of four asymmetric divisions undergone by the sensory organ precursor cells to generate cells that have distinct cell fates. For example, in the external sensory organ, the precursor cells give rise to one multidendritic neuron and four additional cells (the socket, shaft, sheath cells and the external sense neuron). Relationships: is a type of asymmetric cell division [GO:0008356]; is part of sensory organ development [GO:0007423]